prostanoid biosynthetic process [GO:0046457] (biological process) Definition: The chemical reactions and pathways resulting in the formation of prostanoids, any compound based on or derived from the prostanoate structure. Subtypes: prostaglandin biosynthetic process [GO:0001516] Relationships: is_a unsaturated fatty acid biosynthetic process [GO:0006636]; is a type of prostanoid metabolic process [GO:0006692]; is a type of icosanoid biosynthetic process [GO:0046456] Sources: GOC:ai Also known as: prostanoid anabolism, prostanoid biosynthesis, prostanoid formation, prostanoid synthesis